autophagosome organization [GO:1905037] (biological process) Subtypes: autophagosome assembly [GO:0000045], regulation of autophagosome size [GO:0016243], autophagosome membrane disassembly [GO:0030399] Definition: A process that is carried out at the cellular level which results in the assembly, arrangement of constituent parts, or disassembly of an autophagosome. References: PMID:22186024 Sources: GOC:PARL, GOC:TermGenie, GOC:bf Also known as: autophagic vacuole organization, initial autophagic vacuole organization Relationships: is_a GO:0007033; is part of macroautophagy [GO:0016236]